{
  "term_id": "GO:0061844",
  "gene_name": "Ribonuclease K6",
  "gene": "UniProtKB:Q93091",
  "gene_symbol": "RNASE6",
  "term_label": "antimicrobial humoral immune response mediated by antimicrobial peptide"
}